{
  "gene_name": "Nucleolar protein 12",
  "term_id": "UNKNOWN:0002",
  "gene": "UniProtKB:Q9UGY1",
  "term_label": "Unknown biological process",
  "gene_symbol": "NOL12"
}